sensory perception of cold stimulus [GO:0062035] (biological process) References: PMID:21335241 Relationships: is a type of thermoception [GO:0050955] Definition: The series of events required for an organism to receive a cold temperature stimulus, convert it to a molecular signal, and recognize and characterize the signal.